{
  "term_label": "Unknown biological process",
  "gene": "UniProtKB:O43451",
  "term_id": "UNKNOWN:0002",
  "gene_symbol": "MGAM",
  "gene_name": "Maltase-glucoamylase"
}